{
  "gene_name": "Keratin-associated protein 19-4",
  "term_label": "Unknown molecular function",
  "gene_symbol": "KRTAP19-4",
  "term_id": "UNKNOWN:0001",
  "gene": "UniProtKB:Q3LI73"
}